{
  "gene_name": "CASP8-associated protein 2",
  "gene_symbol": "CASP8AP2",
  "term_label": "mitochondrion",
  "term_id": "GO:0005739",
  "gene": "UniProtKB:Q9UKL3"
}